{
  "term_label": "regulation of transcription by RNA polymerase II",
  "gene": "UniProtKB:O75528",
  "gene_symbol": "TADA3",
  "term_id": "GO:0006357",
  "gene_name": "Transcriptional adapter 3"
}